negative regulation of glial cell apoptotic process [GO:0034351] (BP) Subtypes: negative regulation of oligodendrocyte apoptotic process [GO:1900142] Also known as: down regulation of glial cell apoptosis, down-regulation of glial cell apoptosis, downregulation of glial cell apoptosis, inhibition of glial cell apoptosis, negative regulation of glial cell apoptosis Definition: Any process that stops, prevents, or reduces the frequency, rate, or extent of glial cell apoptotic process. Relationships: is a type of regulation of glial cell apoptotic process [GO:0034350]; is a type of GO:0043066; negatively regulates GO:0034349 Sources: GOC:mah, GOC:mtg_apoptosis